{
  "gene_name": "Caveolae-associated protein 1",
  "gene": "UniProtKB:Q6NZI2",
  "term_label": "rRNA primary transcript binding",
  "gene_symbol": "CAVIN1",
  "term_id": "GO:0042134"
}